{
  "term_id": "GO:0019911",
  "term_label": "structural constituent of myelin sheath",
  "gene_name": "Protein MAL2",
  "gene": "UniProtKB:Q969L2",
  "gene_symbol": "MAL2"
}